negative regulation of lateral mesodermal cell fate determination [GO:0048375] (biological process) Sources: GOC:jid Relationships: is_a negative regulation of mesodermal cell fate determination [GO:0048335]; is a type of regulation of lateral mesodermal cell fate determination [GO:0048374]; negatively regulates GO:0048373 Also known as: down regulation of lateral mesodermal cell fate determination, down-regulation of lateral mesodermal cell fate determination, downregulation of lateral mesodermal cell fate determination, negative regulation of lateral plate mesodermal cell fate determination, inhibition of lateral mesodermal cell fate determination Definition: Any process that stops, prevents, or reduces the frequency, rate or extent of lateral mesoderm cell fate determination.